negative regulation of T-helper 1 cell differentiation [GO:0045626] (biological process) Also known as: down regulation of T-helper 1 cell differentiation, down-regulation of T-helper 1 cell differentiation, downregulation of T-helper 1 cell differentiation, inhibition of T-helper 1 cell differentiation, negative regulation of T-helper 1 cell development Note: Note that immunologists typically use the word 'development' to refer to cells of B or T cell lineages undergoing the process that GO describes as 'cell differentiation'. Sources: GOC:go_curators Relationships: is a type of GO:0002826; is_a negative regulation of T-helper cell differentiation [GO:0045623]; is a type of regulation of T-helper 1 cell differentiation [GO:0045625]; negatively regulates T-helper 1 cell differentiation [GO:0045063] Definition: Any process that stops, prevents, or reduces the frequency, rate or extent of T-helper 1 cell differentiation.